{
  "gene_name": "F-box-like_WD repeat-containing protein TBL1XR1",
  "gene_symbol": "TBL1XR1",
  "term_label": "histone deacetylase complex",
  "gene": "UniProtKB:Q9BZK7",
  "term_id": "GO:0000118"
}